L-lysine-lactamase activity [GO:0050028] (molecular function) Also known as: L-alpha-aminocaprolactam hydrolase activity, L-lysinamidase activity, L-lysine-1,6-lactam lactamhydrolase activity Relationships: is a type of hydrolase activity, acting on carbon-nitrogen (but not peptide) bonds, in cyclic amides [GO:0016812] Definition: Catalysis of the reaction: L-2-aminohexano-6-lactam + H2O = L-lysine. Sources: EC:3.5.2.11, RHEA:21388